{
  "term_label": "oligosaccharide metabolic process",
  "gene_symbol": "GLA",
  "term_id": "GO:0009311",
  "gene_name": "Alpha-galactosidase A",
  "gene": "UniProtKB:P06280"
}